{
  "term_label": "transmembrane signaling receptor activity",
  "gene_symbol": "CD300E",
  "term_id": "GO:0004888",
  "gene": "UniProtKB:Q496F6",
  "gene_name": "CMRF35-like molecule 2"
}